{
  "term_label": "Unknown cellular component",
  "gene": "UniProtKB:Q14240",
  "term_id": "UNKNOWN:0003",
  "gene_name": "Eukaryotic initiation factor 4A-II",
  "gene_symbol": "EIF4A2"
}